{
  "gene_name": "Uromodulin-like 1",
  "term_label": "cell surface",
  "term_id": "GO:0009986",
  "gene": "UniProtKB:Q5DID0",
  "gene_symbol": "UMODL1"
}